phosphoglycerate phosphatase activity [GO:0050192] (molecular function) Definition: Catalysis of the reaction: 2-phospho-D-glycerate + H2O = D-glycerate + phosphate. Relationships: is a type of GO:0016791 Sources: EC:3.1.3.20, RHEA:21156 Also known as: D-2-phosphoglycerate phosphatase activity, D-glycerate-2-phosphate phosphohydrolase activity, glycerophosphate phosphatase activity